{
  "term_id": "GO:1902476",
  "gene_symbol": "ANO1",
  "gene_name": "Anoctamin-1",
  "term_label": "chloride transmembrane transport",
  "gene": "UniProtKB:Q5XXA6"
}